regulation of cyclic nucleotide-gated ion channel activity [GO:1902159] (biological process) Also known as: regulation of cyclic nucleotide activated ion channel activity, regulation of cyclic nucleotide gated ion channel activity, regulation of cyclic nucleotide-activated ion channel activity Relationships: is a type of regulation of transmembrane transporter activity [GO:0022898]; regulates cyclic nucleotide-activated monoatomic ion channel activity [GO:0043855] References: PMID:11420311 Sources: GOC:TermGenie Definition: Any process that modulates the frequency, rate or extent of cyclic nucleotide-gated ion channel activity.